{
  "term_id": "GO:0043171",
  "gene_name": "Aminopeptidase Q",
  "term_label": "peptide catabolic process",
  "gene_symbol": "LVRN",
  "gene": "UniProtKB:Q6Q4G3"
}